{
  "gene": "UniProtKB:P63165",
  "gene_name": "Small ubiquitin-related modifier 1",
  "term_label": "PML body",
  "gene_symbol": "SUMO1",
  "term_id": "GO:0016605"
}